{
  "gene_symbol": "NPIPA9",
  "term_label": "Unknown cellular component",
  "gene": "UniProtKB:A0A0B4J1W7",
  "term_id": "UNKNOWN:0003",
  "gene_name": "Nuclear pore complex-interacting protein family member A9"
}